{
  "gene": "UniProtKB:Q3LIE5",
  "gene_name": "Manganese-dependent ADP-ribose_CDP-alcohol diphosphatase",
  "term_id": "UNKNOWN:0003",
  "term_label": "Unknown cellular component",
  "gene_symbol": "ADPRM"
}